virus tail, sheath [GO:0098027] (cellular component) Definition: The external contractile envelope of the tail of some viruses. Its contraction ensures ejection of the virus DNA into the host cytoplasm. Also known as: bacteriophage tail sheath Sources: GOC:bm, VZ:3959 Relationships: is a type of virion component [GO:0044423]; is part of virus tail [GO:0098015]